{
  "term_label": "protein polyubiquitination",
  "gene_symbol": "ERCC8",
  "term_id": "GO:0000209",
  "gene_name": "DNA excision repair protein ERCC-8",
  "gene": "UniProtKB:Q13216"
}